{
  "term_id": "GO:0005856",
  "gene_name": "Leiomodin-2",
  "gene": "UniProtKB:Q6P5Q4",
  "term_label": "cytoskeleton",
  "gene_symbol": "LMOD2"
}